{
  "term_id": "GO:1904158",
  "gene": "UniProtKB:Q4G0P3",
  "term_label": "axonemal central apparatus assembly",
  "gene_symbol": "HYDIN",
  "gene_name": "Hydrocephalus-inducing protein homolog"
}